{
  "gene_symbol": "PTPRA",
  "term_label": "protein tyrosine phosphatase activity",
  "gene_name": "Receptor-type tyrosine-protein phosphatase alpha",
  "gene": "UniProtKB:P18433",
  "term_id": "GO:0004725"
}